4,4-dimethyl-9beta,19-cyclopropylsterol oxidation [GO:0080064] (biological process) Relationships: is_a lipid oxidation [GO:0034440] References: PMID:14653780 Sources: GOC:pr Definition: A lipid oxidation process proceeding through a series of three successive monooxygenations of the alpha methyl group on the C4 carbon (CH3 to CH2OH to CHO to COOH) and resulting in this overall reaction: 4,4-dimethyl-9beta,19-cyclopropylsterol + 3 NADPH + 3 H+ + 3 O2 = 4-alpha-carboxy, 4-beta-methyl-9beta,19-cyclopropylsterol + 3 NADP+ + 3 H2O. Also known as: 4,4-dimethyl-9beta,19-cyclopropylsterol-4alpha-methyl oxidase activity